{
  "term_label": "negative regulation of G protein-coupled receptor signaling pathway",
  "gene_name": "Regulator of G-protein signaling 2",
  "term_id": "GO:0045744",
  "gene_symbol": "RGS2",
  "gene": "UniProtKB:P41220"
}